{
  "term_label": "cytosol",
  "term_id": "GO:0005829",
  "gene": "UniProtKB:O43930",
  "gene_name": "Putative serine_threonine-protein kinase PRKY",
  "gene_symbol": "PRKY"
}